{
  "term_label": "clathrin-coated pit",
  "gene_symbol": "GAS7",
  "term_id": "GO:0005905",
  "gene": "UniProtKB:O60861",
  "gene_name": "Growth arrest-specific protein 7"
}